{
  "term_id": "GO:0004747",
  "gene_name": "Ribokinase",
  "term_label": "ribokinase activity",
  "gene": "UniProtKB:Q9H477",
  "gene_symbol": "RBKS"
}